{
  "term_id": "GO:0005615",
  "term_label": "extracellular space",
  "gene": "UniProtKB:P18075",
  "gene_name": "Bone morphogenetic protein 7",
  "gene_symbol": "BMP7"
}